{
  "gene_name": "Interleukin-18",
  "gene_symbol": "IL18",
  "term_label": "extracellular space",
  "term_id": "GO:0005615",
  "gene": "UniProtKB:Q14116"
}